{
  "gene": "UniProtKB:Q96G61",
  "term_label": "cytoplasm",
  "gene_symbol": "NUDT11",
  "term_id": "GO:0005737",
  "gene_name": "Diphosphoinositol polyphosphate phosphohydrolase 3-beta"
}